{
  "gene_symbol": "SEMA3D",
  "term_id": "GO:0007411",
  "gene_name": "Semaphorin-3D",
  "term_label": "axon guidance",
  "gene": "UniProtKB:O95025"
}